{
  "gene_name": "YTH domain-containing family protein 1",
  "term_label": "stress granule assembly",
  "term_id": "GO:0034063",
  "gene": "UniProtKB:Q9BYJ9",
  "gene_symbol": "YTHDF1"
}